{
  "gene": "UniProtKB:O15327",
  "gene_symbol": "INPP4B",
  "term_label": "Unknown biological process",
  "term_id": "UNKNOWN:0002",
  "gene_name": "Inositol polyphosphate 4-phosphatase type II"
}